nociceptin receptor binding [GO:0031853] (molecular function) Sources: GOC:mah, GOC:nln Also known as: nociceptin receptor ligand Definition: Binding to a nociceptin receptor. Relationships: is a type of opioid receptor binding [GO:0031628]